{
  "gene_symbol": "DNAJB13",
  "gene": "UniProtKB:P59910",
  "term_id": "GO:0051082",
  "gene_name": "DnaJ homolog subfamily B member 13",
  "term_label": "unfolded protein binding"
}